{
  "gene_name": "Ciliogenesis and planar polarity effector 2",
  "gene_symbol": "CPLANE2",
  "term_id": "GO:0035869",
  "term_label": "ciliary transition zone",
  "gene": "UniProtKB:Q9BU20"
}